{
  "gene": "UniProtKB:P56706",
  "gene_symbol": "WNT7B",
  "term_label": "extracellular space",
  "term_id": "GO:0005615",
  "gene_name": "Protein Wnt-7b"
}